{
  "term_label": "chloride transmembrane transport",
  "gene_symbol": "GABRQ",
  "gene_name": "Gamma-aminobutyric acid receptor subunit theta",
  "gene": "UniProtKB:Q9UN88",
  "term_id": "GO:1902476"
}